{
  "term_id": "GO:0003924",
  "gene": "UniProtKB:Q13637",
  "gene_symbol": "RAB32",
  "term_label": "GTPase activity",
  "gene_name": "Ras-related protein Rab-32"
}